inhibitory neuromuscular junction [GO:0098521] (cellular component) Definition: The junction between the axon of a motor neuron and a muscle fiber. In response to the arrival of action potentials, the presynaptic button releases molecules of neurotransmitters into the synaptic cleft. These diffuse across the cleft and transmit the signal to the postsynaptic membrane of the muscle fiber, leading to a change in post-synaptic potential that inhibits muscle contraction. Note: Inhibitory neuromuscular junctions are found in arthropods but not in vertebrates. Subtypes: inhibitory neuromuscular junction of somatic myotube [GO:0098526] Relationships: is a type of neuromuscular junction [GO:0031594]; is a type of inhibitory synapse [GO:0060077] Sources: GOC:dos